positive regulation of butyryl-CoA biosynthetic process from acetyl-CoA [GO:1900496] (biological process) Also known as: activation of butyryl-CoA biosynthesis from acetyl-CoA, positive regulation of butyryl-CoA biosynthesis from acetyl-CoA, up regulation of butyryl-CoA biosynthesis from acetyl-CoA, up regulation of butyryl-CoA biosynthetic process from acetyl-CoA, up-regulation of butyryl-CoA biosynthesis from acetyl-CoA, up-regulation of butyryl-CoA biosynthetic process from acetyl-CoA, upregulation of butyryl-CoA biosynthesis from acetyl-CoA, upregulation of butyryl-CoA biosynthetic process from acetyl-CoA, activation of butyryl-CoA biosynthetic process from acetyl-CoA Sources: GOC:TermGenie, GOC:mengo_curators Definition: Any process that activates or increases the frequency, rate or extent of butyryl-CoA biosynthetic process from acetyl-CoA. Relationships: is a type of positive regulation of amide metabolic process [GO:0034250]; is a type of GO:0045723; is a type of positive regulation of phosphate metabolic process [GO:0045937]; is a type of regulation of butyryl-CoA biosynthetic process from acetyl-CoA [GO:1900494]; RO_0002213 GO:0044579